{
  "term_id": "GO:0008330",
  "gene_name": "Dual specificity protein phosphatase 10",
  "term_label": "protein tyrosine/threonine phosphatase activity",
  "gene": "UniProtKB:Q9Y6W6",
  "gene_symbol": "DUSP10"
}